{
  "term_id": "GO:0007043",
  "gene_name": "Cadherin-24",
  "term_label": "cell-cell junction assembly",
  "gene": "UniProtKB:Q86UP0",
  "gene_symbol": "CDH24"
}